{
  "gene": "UniProtKB:Q8NEA5",
  "term_label": "Unknown molecular function",
  "term_id": "UNKNOWN:0001",
  "gene_symbol": "C19orf18",
  "gene_name": "Uncharacterized protein C19orf18"
}